{
  "term_label": "plus-end-directed vesicle transport along microtubule",
  "gene_name": "FYVE and coiled-coil domain-containing protein 1",
  "gene": "UniProtKB:Q9BQS8",
  "term_id": "GO:0072383",
  "gene_symbol": "FYCO1"
}